{
  "term_id": "GO:0006886",
  "gene_symbol": "SNX27",
  "gene_name": "Sorting nexin-27",
  "term_label": "intracellular protein transport",
  "gene": "UniProtKB:Q96L92"
}